{
  "gene": "UniProtKB:O76070",
  "term_id": "GO:0043025",
  "term_label": "neuronal cell body",
  "gene_name": "Gamma-synuclein",
  "gene_symbol": "SNCG"
}